{
  "gene_symbol": "DDX54",
  "gene": "UniProtKB:Q8TDD1",
  "term_id": "GO:0005730",
  "term_label": "nucleolus",
  "gene_name": "ATP-dependent RNA helicase DDX54"
}